{
  "gene_name": "Transmembrane anterior posterior transformation protein 1 homolog",
  "term_id": "GO:0036064",
  "gene": "UniProtKB:Q6NXT6",
  "term_label": "ciliary basal body",
  "gene_symbol": "TAPT1"
}